{
  "term_id": "GO:0005886",
  "gene": "UniProtKB:Q9Y336",
  "gene_symbol": "SIGLEC9",
  "term_label": "plasma membrane",
  "gene_name": "Sialic acid-binding Ig-like lectin 9"
}